{
  "gene": "UniProtKB:O75607",
  "gene_symbol": "NPM3",
  "gene_name": "Nucleoplasmin-3",
  "term_id": "GO:0042393",
  "term_label": "histone binding"
}